{
  "gene": "UniProtKB:Q9UBX7",
  "gene_name": "Kallikrein-11",
  "gene_symbol": "KLK11",
  "term_id": "GO:0004252",
  "term_label": "serine-type endopeptidase activity"
}